{
  "gene_name": "Family with sequence similarity 90 member A11, pseudogene",
  "term_label": "Unknown biological process",
  "term_id": "UNKNOWN:0002",
  "gene": "UniProtKB:A0A8V8TNH8",
  "gene_symbol": "FAM90A11P"
}